{
  "term_id": "UNKNOWN:0002",
  "gene": "UniProtKB:Q96T59",
  "gene_name": "CMT1A duplicated region transcript 15 protein",
  "gene_symbol": "CDRT15",
  "term_label": "Unknown biological process"
}